regulation of heart rate [GO:0002027] (biological process) References: PMID:10358008 Sources: GOC:dph, GOC:tb Also known as: cardiac chronotropy, regulation of heart contraction rate, regulation of rate of heart contraction Subtypes: circadian regulation of heart rate [GO:0003053], regulation of heart rate by chemical signal [GO:0003062], negative regulation of heart rate [GO:0010459], positive regulation of heart rate [GO:0010460], GO:0086091 Relationships: is a type of regulation of heart contraction [GO:0008016]; is_a GO:0065008 Definition: Any process that modulates the frequency or rate of heart contraction.